{
  "term_id": "GO:0045725",
  "gene": "UniProtKB:Q7L775",
  "term_label": "positive regulation of glycogen biosynthetic process",
  "gene_name": "EPM2A-interacting protein 1",
  "gene_symbol": "EPM2AIP1"
}